{
  "gene": "UniProtKB:Q9GZX7",
  "gene_symbol": "AICDA",
  "gene_name": "Single-stranded DNA cytosine deaminase",
  "term_label": "cytidine to uridine editing",
  "term_id": "GO:0016554"
}